{
  "gene": "UniProtKB:O95201",
  "term_label": "DNA-binding transcription factor activity, RNA polymerase II-specific",
  "gene_symbol": "ZNF205",
  "gene_name": "Transcriptional repressor RHIT",
  "term_id": "GO:0000981"
}